{
  "term_label": "plasma membrane",
  "term_id": "GO:0005886",
  "gene": "UniProtKB:Q9GZW8",
  "gene_name": "Membrane-spanning 4-domains subfamily A member 7",
  "gene_symbol": "MS4A7"
}